{
  "term_label": "apoptotic process",
  "term_id": "GO:0006915",
  "gene": "UniProtKB:Q7Z465",
  "gene_name": "Bcl-2_adenovirus E1B 19 kDa-interacting protein 2-like protein",
  "gene_symbol": "BNIPL"
}